{
  "term_label": "negative regulation of cell cycle",
  "term_id": "GO:0045786",
  "gene": "UniProtKB:O60356",
  "gene_symbol": "NUPR1",
  "gene_name": "Nuclear protein 1"
}